{
  "gene": "UniProtKB:P31639",
  "gene_name": "Sodium_glucose cotransporter 2",
  "gene_symbol": "SLC5A2",
  "term_label": "renal D-glucose absorption",
  "term_id": "GO:0035623"
}